{
  "term_label": "neuropeptide signaling pathway",
  "gene": "UniProtKB:Q9Y271",
  "gene_name": "Cysteinyl leukotriene receptor 1",
  "gene_symbol": "CYSLTR1",
  "term_id": "GO:0007218"
}